{
  "term_label": "plasma membrane",
  "gene_symbol": "CLCN2",
  "term_id": "GO:0005886",
  "gene_name": "Chloride channel protein 2",
  "gene": "UniProtKB:P51788"
}